{
  "gene_symbol": "GAGE2E",
  "term_label": "Unknown molecular function",
  "term_id": "UNKNOWN:0001",
  "gene": "UniProtKB:Q4V326",
  "gene_name": "G antigen 2E"
}